{
  "term_id": "GO:0004984",
  "gene_symbol": "OR4D2",
  "gene_name": "Olfactory receptor 4D2",
  "term_label": "olfactory receptor activity",
  "gene": "UniProtKB:P58180"
}